positive regulation of matrix metallopeptidase secretion [GO:1904466] (biological process) Definition: Any process that activates or increases the frequency, rate or extent of matrix metallopeptidase secretion. Also known as: positive regulation of MMP secretion, up regulation of MMP secretion, up regulation of matrix metallopeptidase secretion, up-regulation of MMP secretion, up-regulation of matrix metallopeptidase secretion, upregulation of MMP secretion, upregulation of matrix metallopeptidase secretion, activation of MMP secretion, activation of matrix metallopeptidase secretion, activation of matrix metalloproteinase secretion, positive regulation of matrix metalloproteinase secretion, up regulation of matrix metalloproteinase secretion, up-regulation of matrix metalloproteinase secretion, upregulation of matrix metalloproteinase secretion Relationships: is a type of positive regulation of protein secretion [GO:0050714]; is a type of regulation of matrix metallopeptidase secretion [GO:1904464]; positively regulates matrix metallopeptidase secretion [GO:1990773] References: PMID:8679543 Sources: GOC:TermGenie, GO_REF:0000058